{
  "gene_name": "Dihydropteridine reductase",
  "term_id": "GO:0006729",
  "gene_symbol": "QDPR",
  "gene": "UniProtKB:P09417",
  "term_label": "tetrahydrobiopterin biosynthetic process"
}